{
  "gene": "UniProtKB:Q9UJQ1",
  "term_label": "establishment of protein localization to organelle",
  "term_id": "GO:0072594",
  "gene_name": "Lysosome-associated membrane glycoprotein 5",
  "gene_symbol": "LAMP5"
}